{
  "gene_symbol": "EXOC3L2",
  "term_label": "Unknown cellular component",
  "gene": "UniProtKB:Q2M3D2",
  "gene_name": "Exocyst complex component 3-like protein 2",
  "term_id": "UNKNOWN:0003"
}